{
  "term_id": "GO:0001734",
  "gene": "UniProtKB:Q86U44",
  "gene_symbol": "METTL3",
  "term_label": "mRNA m(6)A methyltransferase activity",
  "gene_name": "N6-adenosine-methyltransferase catalytic subunit"
}